{
  "term_id": "GO:0000981",
  "gene_name": "Transcription factor COE1",
  "gene_symbol": "EBF1",
  "term_label": "DNA-binding transcription factor activity, RNA polymerase II-specific",
  "gene": "UniProtKB:Q9UH73"
}